regulation of catecholamine uptake involved in synaptic transmission [GO:0051940] (biological process) Sources: GOC:ai Definition: Any process that modulates the frequency, rate or extent of the directed movement of catecholamine neurotransmitters into a neuron or glial cell. Relationships: is a type of regulation of neurotransmitter uptake [GO:0051580]; is_a regulation of amine transport [GO:0051952]; regulates GO:0051934 Subtypes: GO:0051584, positive regulation of catecholamine uptake involved in synaptic transmission [GO:0051944], negative regulation of catecholamine uptake involved in synaptic transmission [GO:0051945] Also known as: regulation of catecholamine uptake during transmission of nerve impulse, regulation of catecholamine neurotransmitter reuptake, regulation of catecholamine neurotransmitter uptake